{
  "gene": "UniProtKB:O15394",
  "gene_symbol": "NCAM2",
  "term_label": "neuron projection",
  "term_id": "GO:0043005",
  "gene_name": "Neural cell adhesion molecule 2"
}